{
  "gene_name": "Ubiquitin carboxyl-terminal hydrolase 17",
  "term_label": "nucleus",
  "gene_symbol": "USP17L2",
  "gene": "UniProtKB:Q6R6M4",
  "term_id": "GO:0005634"
}